{
  "gene_symbol": "ZNF92",
  "gene": "UniProtKB:Q03936",
  "term_label": "regulation of DNA-templated transcription",
  "term_id": "GO:0006355",
  "gene_name": "Zinc finger protein 92"
}